{
  "term_id": "GO:0048663",
  "term_label": "neuron fate commitment",
  "gene": "UniProtKB:Q92858",
  "gene_symbol": "ATOH1",
  "gene_name": "Transcription factor ATOH1"
}